{
  "term_label": "recycling endosome membrane",
  "gene": "UniProtKB:O14828",
  "gene_symbol": "SCAMP3",
  "gene_name": "Secretory carrier-associated membrane protein 3",
  "term_id": "GO:0055038"
}